enzyme activator activity [GO:0008047] (molecular function) Subtypes: GO:0005096, acetyltransferase activator activity [GO:0010698], cyclase activator activity [GO:0010853], GO:0016176, tryptophan hydroxylase activator activity [GO:0016483], peptidase activator activity [GO:0016504], urease activator activity [GO:0018237], GO:0019209, phosphatase activator activity [GO:0019211], sphingolipid activator protein activity [GO:0030290], DNA polymerase processivity factor activity [GO:0030337], tyrosine 3-monooxygenase activator activity [GO:0036470], L-dopa decarboxylase activator activity [GO:0036478], ornithine decarboxylase activator activity [GO:0042978], ribulose-1,5-bisphosphate carboxylase/oxygenase activator activity [GO:0046863], phosphatidylcholine-sterol O-acyltransferase activator activity [GO:0060228], lipase activator activity [GO:0060229], DNA topoisomerase type II (double strand cut, ATP-hydrolyzing) activator activity [GO:0072587], ubiquitin-protein transferase activator activity [GO:0097027], recombinase activator activity [GO:0120230], DNA strand exchange activator activity [GO:0140619], tRNA ligase activator activity [GO:0140733], tRNA methyltransferase activator activity [GO:0141106], guanyl nucleotide exchange factor activator activity [GO:0160124], cyclic nucleotide phosphodiesterase activator activity [GO:0170005], GO:0170008, GO:0170053, polynucleotide adenylyltransferase activator activity [GO:1990749] Also known as: metalloenzyme activator activity Relationships: is a type of enzyme regulator activity [GO:0030234]; is a type of GO:0140677; positively regulates catalytic activity [GO:0003824] Note: This term should only be used in cases when the regulator directly interacts with the enzyme, but does not result in a covalent modification. Sources: GOC:pdt Definition: A molecular function regulator that increases a catalytic activity.